{
  "term_id": "GO:0006511",
  "gene_symbol": "UBQLN3",
  "gene": "UniProtKB:Q9H347",
  "term_label": "ubiquitin-dependent protein catabolic process",
  "gene_name": "Ubiquilin-3"
}